{
  "gene_symbol": "SFTPD",
  "gene": "UniProtKB:P35247",
  "term_id": "GO:0005771",
  "term_label": "multivesicular body",
  "gene_name": "Pulmonary surfactant-associated protein D"
}